isopeptide cross-linking via N6-(L-isoglutamyl)-L-lysine [GO:0018153] (biological process) Definition: The formation of an isopeptide cross-link between peptidyl-lysine and peptidyl-glutamine to produce N6-(L-isoglutamyl)-L-lysine. Relationships: is a type of peptidyl-glutamine modification [GO:0018199]; is a type of peptidyl-lysine modification [GO:0018205]; is a type of isopeptide cross-linking [GO:0018262] Sources: RESID:AA0124